elastin metabolic process [GO:0051541] (biological process) Definition: The chemical reactions and pathways involving elastin, a glycoprotein which is randomly coiled and crosslinked to form elastic fibers that are found in connective tissue. Relationships: is a type of GO:0009100 Sources: GOC:curators Also known as: elastin metabolism Subtypes: elastin catabolic process [GO:0060309]